positive regulation of blood vessel endothelial cell migration [GO:0043536] (biological process) Subtypes: positive regulation of cell migration involved in sprouting angiogenesis [GO:0090050] Relationships: is a type of positive regulation of endothelial cell migration [GO:0010595]; is a type of regulation of blood vessel endothelial cell migration [GO:0043535]; positively regulates GO:0043534 Sources: GOC:go_curators Also known as: up regulation of blood vessel endothelial cell migration, up-regulation of blood vessel endothelial cell migration, upregulation of blood vessel endothelial cell migration, activation of blood vessel endothelial cell migration, stimulation of blood vessel endothelial cell migration Definition: Any process that activates or increases the frequency, rate or extent of the migration of the endothelial cells of blood vessels.